{
  "term_id": "GO:0006606",
  "term_label": "protein import into nucleus",
  "gene": "UniProtKB:Q5SRE5",
  "gene_name": "Nucleoporin NUP188",
  "gene_symbol": "NUP188"
}